{
  "gene_symbol": "PRR19",
  "gene": "UniProtKB:A6NJB7",
  "gene_name": "Proline-rich protein 19",
  "term_id": "UNKNOWN:0001",
  "term_label": "Unknown molecular function"
}